{
  "term_label": "response to steroid hormone",
  "gene": "UniProtKB:P17275",
  "term_id": "GO:0048545",
  "gene_symbol": "JUNB",
  "gene_name": "Transcription factor JunB"
}